{
  "gene_name": "Scm-like with four MBT domains protein 1",
  "gene": "UniProtKB:Q9UHJ3",
  "term_id": "GO:0005634",
  "gene_symbol": "SFMBT1",
  "term_label": "nucleus"
}